endonucleolytic cleavage between LSU-rRNA and 5S rRNA of tricistronic rRNA transcript (SSU-rRNA, LSU-rRNA, 5S) [GO:0000458] (biological process) Definition: Endonucleolytic cleavage to separate a pre-LSU-rRNA from a pre-5S rRNA originally produced as a tricistronic rRNA transcript that contains the Small Subunit (SSU) rRNA, the Large Subunit (LSU) rRNA, and the 5S rRNA, in that order, from 5' to 3' along the primary transcript. Note that the use of the word tricistronic refers only to the number of mature rRNA molecules which will be produced from the primary transcript and ignores tRNAs that may also be present within the primary transcript. Sources: GOC:curators Relationships: is a type of GO:0000449; BFO_0000050 maturation of LSU-rRNA from tricistronic rRNA transcript (SSU-rRNA, LSU-rRNA,5S) [GO:0002108]